{
  "gene_symbol": "LRRC27",
  "term_id": "UNKNOWN:0001",
  "gene": "UniProtKB:Q9C0I9",
  "term_label": "Unknown molecular function",
  "gene_name": "Leucine-rich repeat-containing protein 27"
}